{
  "term_label": "detection of chemical stimulus involved in sensory perception of smell",
  "gene": "UniProtKB:Q6IF00",
  "term_id": "GO:0050911",
  "gene_name": "Olfactory receptor 2T2",
  "gene_symbol": "OR2T2"
}